glucocorticoid catabolic process [GO:0006713] (biological process) Definition: The chemical reactions and pathways resulting in the breakdown of glucocorticoids, hormonal C21 corticosteroids synthesized from cholesterol. Relationships: is a type of steroid catabolic process [GO:0006706]; is a type of glucocorticoid metabolic process [GO:0008211] Also known as: glucocorticoid breakdown, glucocorticoid catabolism, glucocorticoid degradation Sources: ISBN:0198506732 Regulation: regulated by GO:0031949; negatively regulated by GO:0031950; positively regulated by positive regulation of glucocorticoid catabolic process [GO:0031951]